{
  "term_id": "GO:0051604",
  "gene_symbol": "KLK7",
  "gene_name": "Kallikrein-7",
  "term_label": "protein maturation",
  "gene": "UniProtKB:P49862"
}